{
  "gene": "UniProtKB:P0CW27",
  "gene_name": "Coiled-coil domain-containing protein 166",
  "term_label": "Unknown biological process",
  "gene_symbol": "CCDC166",
  "term_id": "UNKNOWN:0002"
}